{
  "term_id": "UNKNOWN:0001",
  "gene_symbol": "PSMB4",
  "gene": "UniProtKB:P28070",
  "gene_name": "Proteasome subunit beta type-4",
  "term_label": "Unknown molecular function"
}